{
  "term_id": "GO:0005085",
  "gene_symbol": "DOCK10",
  "gene": "UniProtKB:Q96BY6",
  "gene_name": "Dedicator of cytokinesis protein 10",
  "term_label": "guanyl-nucleotide exchange factor activity"
}